contractile vacuole dissociation from plasma membrane [GO:0140026] (biological process) References: PMID:22323285 Also known as: contractile vacuole detethering from plasma membrane Definition: The dissociation of the contractile vacuole after discharge, from the plasma membrane. This interaction is mediated by detethering factors that initiate the process of tubulation and fragmentation of the empty contractile vacuole bladder, which is then reincorporated into the CV network. Relationships: is a type of vesicle-mediated transport [GO:0016192]